negative regulation of mitotic spindle assembly checkpoint signaling [GO:0140499] (biological process) Definition: Any process that stops, prevents, or reduces the frequency, rate or extent of negative regulation of mitotic spindle assembly checkpoint signaling. References: PMID:28017606 Subtypes: deactivation of mitotic spindle assembly checkpoint [GO:1902426] Relationships: is a type of GO:0010948; is a type of positive regulation of mitotic metaphase/anaphase transition [GO:0045842]; is a type of positive regulation of mitotic sister chromatid segregation [GO:0062033]; is a type of negative regulation of spindle checkpoint [GO:0090233]; is a type of regulation of mitotic cell cycle spindle assembly checkpoint [GO:0090266]; negatively regulates mitotic spindle assembly checkpoint signaling [GO:0007094]